{
  "term_id": "GO:0140566",
  "gene_symbol": "BRPF3",
  "gene": "UniProtKB:Q9ULD4",
  "term_label": "histone reader activity",
  "gene_name": "Bromodomain and PHD finger-containing protein 3"
}